{
  "term_label": "transcription corepressor activity",
  "term_id": "GO:0003714",
  "gene_name": "DNA-binding protein inhibitor ID-4",
  "gene_symbol": "ID4",
  "gene": "UniProtKB:P47928"
}